{
  "gene": "UniProtKB:Q9H093",
  "term_label": "cellular response to glucose starvation",
  "term_id": "GO:0042149",
  "gene_symbol": "NUAK2",
  "gene_name": "NUAK family SNF1-like kinase 2"
}